{
  "term_id": "GO:0005549",
  "gene": "UniProtKB:Q8TDV2",
  "gene_symbol": "GPR148",
  "term_label": "odorant binding",
  "gene_name": "Probable G-protein coupled receptor 148"
}